{
  "gene_symbol": "ZNF793",
  "term_label": "DNA-binding transcription factor activity, RNA polymerase II-specific",
  "gene": "UniProtKB:Q6ZN11",
  "gene_name": "Zinc finger protein 793",
  "term_id": "GO:0000981"
}